{
  "term_id": "UNKNOWN:0002",
  "gene_symbol": "OR51F2",
  "gene": "UniProtKB:Q8NH61",
  "gene_name": "Olfactory receptor 51F2",
  "term_label": "Unknown biological process"
}